progesterone metabolic process [GO:0042448] (biological process) Definition: The chemical reactions and pathways involving progesterone, a steroid hormone produced in the ovary which prepares and maintains the uterus for pregnancy. Also found in plants. Subtypes: progesterone biosynthetic process [GO:0006701], GO:0006709 Relationships: is a type of GO:0008207; is a type of ketone metabolic process [GO:0042180]; is a type of olefinic compound metabolic process [GO:0120254] Also known as: progesterone metabolism References: PMID:11392024 Sources: GOC:jl